{
  "gene_symbol": "H1-4",
  "gene": "UniProtKB:P10412",
  "term_id": "GO:0000791",
  "gene_name": "Histone H1.4",
  "term_label": "euchromatin"
}